{
  "gene": "UniProtKB:Q2M1P5",
  "term_id": "GO:0007018",
  "gene_symbol": "KIF7",
  "gene_name": "Kinesin-like protein KIF7",
  "term_label": "microtubule-based movement"
}